{
  "gene_name": "Alcohol dehydrogenase 1C",
  "term_label": "zinc ion binding",
  "term_id": "GO:0008270",
  "gene_symbol": "ADH1C",
  "gene": "UniProtKB:P00326"
}